{
  "gene_name": "Coiled-coil domain-containing protein 14",
  "gene_symbol": "CCDC14",
  "gene": "UniProtKB:Q49A88",
  "term_label": "protein localization to centrosome",
  "term_id": "GO:0071539"
}